mitotic G2 cell size control checkpoint signaling [GO:0031569] (biological process) Definition: A signal transduction process that contributes to a cell size control checkpoint prior to the G2/M transition of mitosis. Sources: GOC:mtg_cell_cycle Also known as: G2 cell size control checkpoint, G2/M transition size control checkpoint, mitotic cell cycle G2/M transition size control checkpoint, mitotic G2 cell size control checkpoint, signal transduction involved in G2 cell size control checkpoint, signal transduction involved in G2/M transition size control checkpoint, signal transduction involved in mitotic cell cycle G2/M transition size control checkpoint Relationships: is a type of negative regulation of G2/M transition of mitotic cell cycle [GO:0010972]; is_a GO:0031567; happens during GO:0051319